{
  "gene": "UniProtKB:P41595",
  "gene_symbol": "HTR2B",
  "term_id": "GO:0005886",
  "gene_name": "5-hydroxytryptamine receptor 2B",
  "term_label": "plasma membrane"
}